sphingosine catabolic process [GO:0051872] (biological process) Definition: The chemical reactions and pathways resulting in the breakdown of sphingosine (sphing-4-enine), trans-D-erytho-2-amino-octadec-4-ene-1,3-diol, a long chain amino diol sphingoid base that occurs in most sphingolipids in animal tissues. Relationships: is a type of sphingosine metabolic process [GO:0006670]; is a type of GO:0034313; is a type of sphingoid catabolic process [GO:0046521] Sources: GOC:ai Also known as: (4E)-sphing-4-enine catabolic process, (4E)-sphing-4-enine catabolism, sphing-4-enine catabolic process, sphing-4-enine catabolism